{
  "gene": "UniProtKB:Q8IUX7",
  "gene_name": "Adipocyte enhancer-binding protein 1",
  "term_label": "RNA polymerase II transcription regulatory region sequence-specific DNA binding",
  "gene_symbol": "AEBP1",
  "term_id": "GO:0000977"
}